{
  "term_label": "small GTPase binding",
  "gene_symbol": "RILP",
  "gene": "UniProtKB:Q96NA2",
  "term_id": "GO:0031267",
  "gene_name": "Rab-interacting lysosomal protein"
}